{
  "gene_symbol": "HLA-DQB2",
  "term_label": "antigen processing and presentation of exogenous peptide antigen via MHC class II",
  "term_id": "GO:0019886",
  "gene": "UniProtKB:P05538",
  "gene_name": "HLA class II histocompatibility antigen, DQ beta 2 chain"
}